positive regulation of sarcinapterin biosynthetic process [GO:1900973] (biological process) Also known as: activation of sarcinapterin anabolism, activation of sarcinapterin biosynthesis, activation of sarcinapterin formation, activation of sarcinapterin synthesis, positive regulation of sarcinapterin anabolism, positive regulation of sarcinapterin biosynthesis, positive regulation of sarcinapterin formation, positive regulation of sarcinapterin synthesis, up regulation of sarcinapterin anabolism, up regulation of sarcinapterin biosynthesis, up regulation of sarcinapterin biosynthetic process, up regulation of sarcinapterin formation, up regulation of sarcinapterin synthesis, up-regulation of sarcinapterin anabolism, up-regulation of sarcinapterin biosynthesis, up-regulation of sarcinapterin biosynthetic process, up-regulation of sarcinapterin formation, up-regulation of sarcinapterin synthesis, upregulation of sarcinapterin anabolism, upregulation of sarcinapterin biosynthesis, upregulation of sarcinapterin biosynthetic process, upregulation of sarcinapterin formation, upregulation of sarcinapterin synthesis, activation of sarcinapterin biosynthetic process Sources: GOC:TermGenie, GOC:mengo_curators Definition: Any process that activates or increases the frequency, rate or extent of sarcinapterin biosynthetic process. Relationships: is a type of positive regulation of biosynthetic process [GO:0009891]; is a type of GO:0045937; is a type of positive regulation of small molecule metabolic process [GO:0062013]; is a type of regulation of sarcinapterin biosynthetic process [GO:1900971]; positively regulates sarcinapterin biosynthetic process [GO:1900868]